{
  "term_label": "Unknown cellular component",
  "term_id": "UNKNOWN:0003",
  "gene": "UniProtKB:A6NEQ2",
  "gene_name": "Protein FAM181B",
  "gene_symbol": "FAM181B"
}